{
  "gene_name": "Salivary gland specific protein SAGSIN1",
  "gene_symbol": "SAGSIN1",
  "gene": "UniProtKB:A0A0C4DGP1",
  "term_id": "UNKNOWN:0001",
  "term_label": "Unknown molecular function"
}